{
  "term_id": "UNKNOWN:0002",
  "gene": "UniProtKB:A0A1W2PRN1",
  "term_label": "Unknown biological process",
  "gene_name": "Golgin subfamily A conserved domain-containing protein",
  "gene_symbol": "A0A1W2PRN1"
}